{
  "gene": "UniProtKB:Q92830",
  "term_label": "histone H3 acetyltransferase activity",
  "gene_name": "Histone acetyltransferase KAT2A",
  "term_id": "GO:0010484",
  "gene_symbol": "KAT2A"
}